{
  "term_label": "spindle pole",
  "term_id": "GO:0000922",
  "gene": "UniProtKB:Q9H4B4",
  "gene_symbol": "PLK3",
  "gene_name": "Serine_threonine-protein kinase PLK3"
}